{
  "gene_name": "Elongation factor G, mitochondrial",
  "gene_symbol": "GFM1",
  "term_id": "GO:0070125",
  "gene": "UniProtKB:Q96RP9",
  "term_label": "mitochondrial translational elongation"
}